{
  "term_label": "serine C-palmitoyltransferase activity",
  "gene": "UniProtKB:O15270",
  "gene_name": "Serine palmitoyltransferase 2",
  "gene_symbol": "SPTLC2",
  "term_id": "GO:0004758"
}